{
  "term_label": "innate immune response in mucosa",
  "gene_name": "Histone H2B type 1-L",
  "gene": "UniProtKB:Q99880",
  "gene_symbol": "H2BC13",
  "term_id": "GO:0002227"
}